{
  "gene_name": "Contactin-6",
  "term_id": "GO:0045202",
  "gene": "UniProtKB:Q9UQ52",
  "term_label": "synapse",
  "gene_symbol": "CNTN6"
}